mannitol metabolic process [GO:0019594] (biological process) Sources: ISBN:0198506732 Also known as: mannitol metabolism Subtypes: mannitol catabolic process [GO:0019592], mannitol biosynthetic process [GO:0019593] Definition: The chemical reactions and pathways involving mannitol, the alditol derived from D-mannose by reduction of the aldehyde group. Relationships: is_a GO:0006059